{
  "gene": "UniProtKB:Q9UIB8",
  "gene_symbol": "CD84",
  "term_label": "T cell activation",
  "term_id": "GO:0042110",
  "gene_name": "SLAM family member 5"
}